maturation of LSU-rRNA from tricistronic rRNA transcript (SSU-rRNA, LSU-rRNA,5S) [GO:0002108] (biological process) Definition: Any process involved in the maturation of a precursor Large SubUnit (LSU) ribosomal RNA (rRNA) molecule into a mature LSU-rRNA molecule from the pre-rRNA molecule originally produced as a tricistronic rRNA transcript that contains the Small Subunit (SSU) rRNA, Large Subunit (LSU) the 5S rRNA in that order from 5' to 3' along the primary transcript. Relationships: is a type of maturation of LSU-rRNA [GO:0000470] Sources: GOC:curators